plastid gene expression [GO:0140899] (biological process) Definition: The process in which a plastid gene's sequence is converted into a mature gene product or products (proteins or RNA). This includes the production of an RNA transcript as well as any processing to produce a mature RNA product or an mRNA or circRNA (for protein-coding genes) and the translation of that mRNA or circRNA into protein. Protein maturation is included when required to form an active form of a product from an inactive precursor form. Relationships: is a type of gene expression [GO:0010467]; occurs in plastid [GO:0009536] References: PMID:28377785